{
  "gene": "UniProtKB:Q9Y5P3",
  "term_label": "animal organ development",
  "gene_symbol": "RAI2",
  "gene_name": "Retinoic acid-induced protein 2",
  "term_id": "GO:0048513"
}